{
  "gene": "UniProtKB:Q9BSM1",
  "term_id": "GO:1990841",
  "term_label": "promoter-specific chromatin binding",
  "gene_symbol": "PCGF1",
  "gene_name": "Polycomb group RING finger protein 1"
}